{
  "gene": "UniProtKB:P37231",
  "term_id": "GO:0009755",
  "term_label": "hormone-mediated signaling pathway",
  "gene_name": "Peroxisome proliferator-activated receptor gamma",
  "gene_symbol": "PPARG"
}